{
  "term_id": "GO:0030198",
  "gene": "UniProtKB:P45452",
  "gene_symbol": "MMP13",
  "gene_name": "Collagenase 3",
  "term_label": "extracellular matrix organization"
}